L-asparagine biosynthetic process [GO:0070981] (biological process) Also known as: L-asparagine anabolism, L-asparagine biosynthesis, L-asparagine formation, L-asparagine synthesis Definition: The chemical reactions and pathways resulting in the formation of asparagine, (2S)-2-amino-3-carbamoylpropanoic acid. Sources: GOC:mah Subtypes: L-asparagine biosynthetic process from oxaloacetate [GO:0019266], GO:0019267 Relationships: is a type of aspartate family amino acid biosynthetic process [GO:0009067]; is a type of amide biosynthetic process [GO:0043604]; is a type of L-asparagine metabolic process [GO:0070982]